{
  "term_label": "G protein-coupled receptor signaling pathway",
  "gene": "UniProtKB:P63218",
  "term_id": "GO:0007186",
  "gene_symbol": "GNG5",
  "gene_name": "Guanine nucleotide-binding protein G(I)_G(S)_G(O) subunit gamma-5"
}